{
  "gene": "UniProtKB:P0DMP1",
  "gene_symbol": "MTRNR2L12",
  "term_label": "Unknown molecular function",
  "gene_name": "Humanin-like 12",
  "term_id": "UNKNOWN:0001"
}